{
  "term_label": "cytosol",
  "gene_name": "EKC_KEOPS complex subunit TPRKB",
  "gene_symbol": "TPRKB",
  "gene": "UniProtKB:Q9Y3C4",
  "term_id": "GO:0005829"
}